{
  "gene": "UniProtKB:Q6VEQ5",
  "gene_symbol": "WASH2P",
  "gene_name": "WAS protein family homolog 2",
  "term_label": "endocytic recycling",
  "term_id": "GO:0032456"
}